geranylgeranyl diphosphate metabolic process [GO:0033385] (biological process) Definition: The chemical reactions and pathways involving geranylgeranyl diphosphate, a polyprenol compound involved in the biosynthesis of a variety of terpenoids including chlorophylls, carotenoids, tocopherols, plastoquinones, and the plant hormones gibberellins. Also known as: geranylgeranyl diphosphate metabolism, geranylgeranyldiphosphate metabolic process Sources: GOC:mah Relationships: is_a phospholipid metabolic process [GO:0006644]; is a type of terpenoid metabolic process [GO:0006721] Subtypes: GO:0033386, geranylgeranyl diphosphate catabolic process [GO:1902247]